negative regulation of zygosporangium development [GO:0075274] (biological process) Definition: Any process that stops, prevents, or reduces the frequency, rate or extent of zygosporangium development, a process in which a fruiting body called zygosporangium is formed. Relationships: is a type of negative regulation of spore-bearing organ development [GO:0075262]; is a type of regulation of zygosporangium development [GO:0075272]; negatively regulates GO:0075271 Sources: GOC:pamgo_curators